{
  "gene_name": "Homogentisate 1,2-dioxygenase",
  "gene": "UniProtKB:Q93099",
  "gene_symbol": "HGD",
  "term_label": "Unknown cellular component",
  "term_id": "UNKNOWN:0003"
}